{
  "term_label": "Unknown molecular function",
  "term_id": "UNKNOWN:0001",
  "gene_name": "T cell receptor alpha variable 9-1",
  "gene_symbol": "TRAV9-1",
  "gene": "UniProtKB:A0A075B6T8"
}